{
  "gene_symbol": "OR51E1",
  "gene_name": "Olfactory receptor 51E1",
  "term_label": "olfactory receptor activity",
  "term_id": "GO:0004984",
  "gene": "UniProtKB:Q8TCB6"
}